{
  "gene_name": "Cation channel sperm-associated auxiliary subunit delta",
  "term_id": "UNKNOWN:0001",
  "term_label": "Unknown molecular function",
  "gene": "UniProtKB:Q86XM0",
  "gene_symbol": "CATSPERD"
}